determination of sensory modality [GO:0050887] (biological process) Definition: The determination of the type or quality of a sensation. Sensory modalities include touch, thermal sensation, visual sensation, auditory sensation and pain. Relationships: is a type of sensory processing [GO:0050893] Sources: ISBN:0721619908